{
  "term_id": "UNKNOWN:0001",
  "gene_name": "Coiled-coil domain-containing protein 179",
  "gene": "UniProtKB:H3BU77",
  "term_label": "Unknown molecular function",
  "gene_symbol": "CCDC179"
}